{
  "term_id": "UNKNOWN:0001",
  "gene_symbol": "HMBOX1",
  "gene_name": "Homeobox-containing protein 1",
  "term_label": "Unknown molecular function",
  "gene": "UniProtKB:Q6NT76"
}